{
  "gene_symbol": "PCDHAC2",
  "gene": "UniProtKB:Q9Y5I4",
  "term_id": "GO:0050839",
  "term_label": "cell adhesion molecule binding",
  "gene_name": "Protocadherin alpha-C2"
}